{
  "term_label": "Unknown biological process",
  "gene_symbol": "ANKRD20A3P",
  "term_id": "UNKNOWN:0002",
  "gene_name": "Putative ankyrin repeat domain-containing protein 20A3",
  "gene": "UniProtKB:Q5VUR7"
}